{
  "term_label": "nucleus",
  "gene_symbol": "DRGX",
  "gene_name": "Dorsal root ganglia homeobox protein",
  "term_id": "GO:0005634",
  "gene": "UniProtKB:A6NNA5"
}